{
  "gene_name": "Ras-related C3 botulinum toxin substrate 3",
  "term_id": "GO:1902622",
  "gene": "UniProtKB:P60763",
  "term_label": "regulation of neutrophil migration",
  "gene_symbol": "RAC3"
}